{
  "gene_symbol": "ERAS",
  "term_label": "positive regulation of cell population proliferation",
  "gene": "UniProtKB:Q7Z444",
  "term_id": "GO:0008284",
  "gene_name": "GTPase ERas"
}